{
  "gene_name": "Melanopsin",
  "gene": "UniProtKB:Q9UHM6",
  "term_id": "GO:0005886",
  "term_label": "plasma membrane",
  "gene_symbol": "OPN4"
}